{
  "gene_symbol": "NEXN-AS1",
  "gene_name": "Putative uncharacterized protein NEXN-AS1",
  "term_label": "Unknown cellular component",
  "term_id": "UNKNOWN:0003",
  "gene": "UniProtKB:Q8NBZ9"
}